{
  "gene_symbol": "PRDX2",
  "term_label": "response to oxidative stress",
  "gene_name": "Peroxiredoxin-2",
  "gene": "UniProtKB:P32119",
  "term_id": "GO:0006979"
}